{
  "term_id": "GO:1901800",
  "gene_name": "Endothelial cell-specific chemotaxis regulator",
  "gene": "UniProtKB:Q19T08",
  "gene_symbol": "ECSCR",
  "term_label": "positive regulation of proteasomal protein catabolic process"
}